{
  "term_id": "GO:0051132",
  "gene_name": "C-type lectin domain family 2 member B",
  "term_label": "NK T cell activation",
  "gene_symbol": "CLEC2B",
  "gene": "UniProtKB:Q92478"
}